{
  "gene": "UniProtKB:Q9BXQ6",
  "gene_name": "Transmembrane protein 121B",
  "term_id": "UNKNOWN:0001",
  "term_label": "Unknown molecular function",
  "gene_symbol": "TMEM121B"
}